{
  "term_id": "GO:0005525",
  "gene_symbol": "TUBE1",
  "gene": "UniProtKB:Q9UJT0",
  "term_label": "GTP binding",
  "gene_name": "Tubulin epsilon chain"
}